inaD signaling complex [GO:0016027] (cellular component) Relationships: is a type of plasma membrane protein complex [GO:0098797]; is part of rhabdomere [GO:0016028]; BFO_0000050 extrinsic component of plasma membrane [GO:0019897] Also known as: inaD signalling complex References: PMID:9010208, PMID:9796815 Sources: GOC:hb Definition: A complex of proteins that are involved in phototransduction and attached to the transient receptor potential (TRP) channel. The protein connections are mediated through inaD.